{
  "term_label": "S-adenosylhomocysteine metabolic process",
  "gene_name": "Glycine N-methyltransferase",
  "term_id": "GO:0046498",
  "gene": "UniProtKB:Q14749",
  "gene_symbol": "GNMT"
}